{
  "gene_name": "Zinc finger protein 483",
  "term_id": "GO:0000978",
  "term_label": "RNA polymerase II cis-regulatory region sequence-specific DNA binding",
  "gene": "UniProtKB:Q8TF39",
  "gene_symbol": "ZNF483"
}